{
  "gene_name": "Protein-tyrosine sulfotransferase 2",
  "term_label": "Golgi apparatus",
  "term_id": "GO:0005794",
  "gene_symbol": "TPST2",
  "gene": "UniProtKB:O60704"
}